{
  "term_id": "GO:0042797",
  "gene_symbol": "POLR2L",
  "gene": "UniProtKB:P62875",
  "gene_name": "DNA-directed RNA polymerases I, II, and III subunit RPABC5",
  "term_label": "tRNA transcription by RNA polymerase III"
}